{
  "gene_symbol": "ADGRL3",
  "term_label": "glutamatergic synapse",
  "term_id": "GO:0098978",
  "gene_name": "Adhesion G protein-coupled receptor L3",
  "gene": "UniProtKB:Q9HAR2"
}